G-protein alpha(q)-synembrin complex [GO:0071152] (cellular component) Relationships: is a type of intracellular protein-containing complex [GO:0140535]; BFO_0000050 intracellular anatomical structure [GO:0005622] References: PMID:12509430 Sources: GOC:mah Also known as: Ric-8A G(q) alpha subunit complex Definition: A protein complex formed by the association of the guanine nucleotide exchange factor synembrin with the alpha(q) subunit of a heterotrimeric G protein.